{
  "gene": "UniProtKB:P16234",
  "gene_symbol": "PDGFRA",
  "term_id": "GO:0005886",
  "term_label": "plasma membrane",
  "gene_name": "Platelet-derived growth factor receptor alpha"
}